{
  "term_id": "GO:0015369",
  "gene": "UniProtKB:O95202",
  "term_label": "calcium:proton antiporter activity",
  "gene_name": "Mitochondrial proton_calcium exchanger protein",
  "gene_symbol": "LETM1"
}